{
  "gene_symbol": "SLX9",
  "gene": "UniProtKB:Q9NSI2",
  "term_label": "Unknown cellular component",
  "term_id": "UNKNOWN:0003",
  "gene_name": "Ribosome biogenesis protein SLX9 homolog"
}